{
  "gene": "UniProtKB:A5YKK6",
  "gene_name": "CCR4-NOT transcription complex subunit 1",
  "term_label": "CCR4-NOT core complex",
  "gene_symbol": "CNOT1",
  "term_id": "GO:0030015"
}